regulation of hepatocyte differentiation [GO:0070366] (biological process) Definition: Any process that modulates the frequency, rate or extent of hepatocyte differentiation. Sources: GOC:mah, GOC:sl Also known as: regulation of liver cell differentiation Relationships: is a type of GO:0030856; regulates GO:0070365 Subtypes: GO:0070367, positive regulation of hepatocyte differentiation [GO:0070368]